{
  "gene_name": "Spermatogenesis-associated protein 25",
  "term_id": "UNKNOWN:0001",
  "gene_symbol": "SPATA25",
  "term_label": "Unknown molecular function",
  "gene": "UniProtKB:Q9BR10"
}